cytosolic proteasome core complex, alpha-subunit complex [GO:0031606] (cellular component) Definition: The proteasome core subcomplex that constitutes the two outer rings of the cytosolic proteasome core complex. Sources: GOC:mah, GOC:mtg_sensu Relationships: is a type of proteasome core complex, alpha-subunit complex [GO:0019773]; is part of cytosolic proteasome core complex [GO:0031603]